{
  "gene": "UniProtKB:Q9NZC4",
  "gene_name": "ETS homologous factor",
  "term_label": "regulation of transcription by RNA polymerase II",
  "gene_symbol": "EHF",
  "term_id": "GO:0006357"
}